positive regulation of nervous system process [GO:0031646] (biological process) Also known as: positive regulation of neurological process, positive regulation of neurological system process, positive regulation of neurophysiological process, up regulation of neurological process, up-regulation of neurological process, upregulation of neurological process, activation of neurological process, stimulation of neurological process Sources: GOC:dph, GOC:mah, GOC:tb Subtypes: positive regulation of myelination [GO:0031643], positive regulation of transmission of nerve impulse [GO:0051971], GO:0097151, positive regulation of sensory perception of pain [GO:1904058], positive regulation of sensory perception of sweet taste [GO:1904658], GO:1904662, GO:1905789 Definition: Any process that activates or increases the frequency, rate or extent of a neurophysiological process. Relationships: is a type of GO:0031644; is_a GO:0051240; positively regulates nervous system process [GO:0050877]